maintenance of protein location in chloroplast [GO:0072597] (biological process) Definition: Any process in which a protein is maintained in a specific location in a chloroplast, and is prevented from moving elsewhere. Relationships: is_a maintenance of protein localization in organelle [GO:0072595]; is part of GO:0072598; occurs in chloroplast [GO:0009507] Sources: GOC:mah